{
  "term_id": "GO:0019432",
  "gene_symbol": "LPIN3",
  "gene_name": "Phosphatidate phosphatase LPIN3",
  "term_label": "triglyceride biosynthetic process",
  "gene": "UniProtKB:Q9BQK8"
}